{
  "gene": "UniProtKB:P48067",
  "gene_symbol": "SLC6A9",
  "term_label": "plasma membrane",
  "gene_name": "Sodium- and chloride-dependent glycine transporter 1",
  "term_id": "GO:0005886"
}